glycine C-acetyltransferase activity [GO:0008890] (molecular function) Relationships: is a type of C-acetyltransferase activity [GO:0016453] Sources: EC:2.3.1.29, RHEA:20736 Also known as: glycine acetyltransferase activity Definition: Catalysis of the reaction: acetyl-CoA + glycine = L-2-amino-3-oxobutanoate + CoA.